{
  "gene_name": "Coiled-coil domain-containing protein 177",
  "term_id": "UNKNOWN:0001",
  "gene_symbol": "CCDC177",
  "gene": "UniProtKB:Q9NQR7",
  "term_label": "Unknown molecular function"
}